{
  "gene_symbol": "RPL18A",
  "term_id": "GO:0002181",
  "gene": "UniProtKB:Q02543",
  "term_label": "cytoplasmic translation",
  "gene_name": "Large ribosomal subunit protein eL20"
}